{
  "gene": "UniProtKB:Q9H7V2",
  "gene_symbol": "SYNDIG1",
  "term_label": "Unknown molecular function",
  "gene_name": "Synapse differentiation-inducing gene protein 1",
  "term_id": "UNKNOWN:0001"
}